{
  "term_label": "Unknown biological process",
  "term_id": "UNKNOWN:0002",
  "gene_symbol": "TSPAN15",
  "gene_name": "Tetraspanin-15",
  "gene": "UniProtKB:O95858"
}